{
  "term_label": "serine-type endopeptidase activity",
  "gene_symbol": "HPR",
  "gene_name": "Haptoglobin-related protein",
  "gene": "UniProtKB:P00739",
  "term_id": "GO:0004252"
}